{
  "term_id": "GO:0000139",
  "term_label": "Golgi membrane",
  "gene_name": "Protein TMEPAI",
  "gene": "UniProtKB:Q969W9",
  "gene_symbol": "PMEPA1"
}